amyloid precursor protein metabolic process [GO:0042982] (biological process) Definition: The chemical reactions and pathways involving amyloid precursor protein (APP), the precursor of amyloid-beta, a glycoprotein associated with Alzheimer's disease. Sources: GOC:go_curators Also known as: APP metabolic process, APP metabolism, amyloid precursor protein metabolism Relationships: is a type of protein metabolic process [GO:0019538] Subtypes: amyloid precursor protein biosynthetic process [GO:0042983], amyloid precursor protein catabolic process [GO:0042987]